{
  "gene_symbol": "IFNL2",
  "gene": "UniProtKB:Q8IZJ0",
  "gene_name": "Interferon lambda-2",
  "term_label": "signaling receptor binding",
  "term_id": "GO:0005102"
}